positive regulation of muscle atrophy [GO:0014737] (biological process) Sources: GOC:mtg_muscle Definition: Any process that activates or increases the frequency, rate or extent of muscle atrophy. Relationships: is a type of GO:0014735; is_a GO:0014744; positively regulates GO:0014889